{
  "gene": "UniProtKB:P05556",
  "gene_name": "Integrin beta-1",
  "term_label": "cell-cell adhesion",
  "term_id": "GO:0098609",
  "gene_symbol": "ITGB1"
}